{
  "term_label": "BAD-BCL-2 complex",
  "gene_name": "Bcl2-associated agonist of cell death",
  "term_id": "GO:0097138",
  "gene": "UniProtKB:Q92934",
  "gene_symbol": "BAD"
}